{
  "gene_name": "PRAME family member 2",
  "gene": "UniProtKB:O60811",
  "term_id": "GO:0031462",
  "gene_symbol": "PRAMEF2",
  "term_label": "Cul2-RING ubiquitin ligase complex"
}